{
  "gene": "UniProtKB:P05937",
  "term_id": "UNKNOWN:0002",
  "term_label": "Unknown biological process",
  "gene_symbol": "CALB1",
  "gene_name": "Calbindin"
}